{
  "term_id": "GO:0045944",
  "gene": "UniProtKB:O60264",
  "term_label": "positive regulation of transcription by RNA polymerase II",
  "gene_symbol": "SMARCA5",
  "gene_name": "SWI_SNF-related matrix-associated actin-dependent regulator of chromatin subfamily A member 5"
}